{
  "gene": "UniProtKB:Q96LT6",
  "gene_symbol": "C1orf74",
  "term_label": "Unknown biological process",
  "gene_name": "UPF0739 protein C1orf74",
  "term_id": "UNKNOWN:0002"
}